{
  "term_id": "UNKNOWN:0003",
  "term_label": "Unknown cellular component",
  "gene_name": "Putative short-chain dehydrogenase_reductase family 42E member 2",
  "gene_symbol": "SDR42E2",
  "gene": "UniProtKB:A6NKP2"
}